{
  "term_id": "UNKNOWN:0001",
  "gene_name": "Methylosome subunit pICln",
  "gene_symbol": "CLNS1A",
  "gene": "UniProtKB:P54105",
  "term_label": "Unknown molecular function"
}